{
  "gene_name": "Protein RIC-3",
  "term_id": "GO:0034394",
  "term_label": "protein localization to cell surface",
  "gene_symbol": "RIC3",
  "gene": "UniProtKB:Q7Z5B4"
}